{
  "term_id": "UNKNOWN:0001",
  "term_label": "Unknown molecular function",
  "gene": "UniProtKB:Q8N9N8",
  "gene_symbol": "EIF1AD",
  "gene_name": "Probable RNA-binding protein EIF1AD"
}